{
  "gene_name": "4-trimethylaminobutyraldehyde dehydrogenase",
  "term_label": "4-trimethylammoniobutyraldehyde dehydrogenase activity",
  "gene": "UniProtKB:P49189",
  "gene_symbol": "ALDH9A1",
  "term_id": "GO:0047105"
}